{
  "gene_name": "Putative PIN1-like protein",
  "term_id": "UNKNOWN:0001",
  "gene": "UniProtKB:O15428",
  "term_label": "Unknown molecular function",
  "gene_symbol": "PIN1P1"
}